negative regulation of bone trabecula formation [GO:1900155] (biological process) Definition: Any process that stops, prevents or reduces the frequency, rate or extent of bone trabecula formation. Sources: GOC:BHF, GOC:TermGenie Also known as: down regulation of bone trabecula formation, down regulation of bone trabeculation, down regulation of skeletal trabecula formation, down regulation of skeletal trabeculation, down-regulation of bone trabecula formation, down-regulation of bone trabeculation, down-regulation of skeletal trabecula formation, down-regulation of skeletal trabeculation, downregulation of bone trabecula formation, downregulation of bone trabeculation, downregulation of skeletal trabecula formation, downregulation of skeletal trabeculation, negative regulation of bone trabeculation, negative regulation of skeletal trabecula formation, negative regulation of skeletal trabeculation, inhibition of bone trabecula formation, inhibition of bone trabeculation, inhibition of skeletal trabecula formation, inhibition of skeletal trabeculation, down regulation of bone trabecula biogenesis, down regulation of skeletal trabecula biogenesis, down-regulation of bone trabecula biogenesis, down-regulation of skeletal trabecula biogenesis, downregulation of bone trabecula biogenesis, downregulation of skeletal trabecula biogenesis, inhibition of bone trabecula biogenesis, inhibition of skeletal trabecula biogenesis, negative regulation of bone trabecula biogenesis, negative regulation of skeletal trabecula biogenesis Relationships: is a type of negative regulation of developmental process [GO:0051093]; is a type of regulation of bone trabecula formation [GO:1900154]; RO_0002212 bone trabecula formation [GO:0060346]